trehalose biosynthetic process [GO:0005992] (biological process) Relationships: is_a trehalose metabolic process [GO:0005991]; is a type of disaccharide biosynthetic process [GO:0046351] Definition: The chemical reactions and pathways resulting in the formation of trehalose, a disaccharide that consists of two molecules of glucose and is isomeric with sucrose. Also known as: mycose biosynthesis, mycose biosynthetic process, mykose biosynthesis, mykose biosynthetic process, trehalose anabolism, trehalose biosynthesis, trehalose formation, trehalose synthesis Sources: GOC:jl, ISBN:0028623819